hyaline layer [GO:0033166] (cellular component) Relationships: is a type of GO:0140047 References: PMID:1721506, PMID:9473317 Definition: A multilayered extraembryonic matrix that functions as a substrate for cell adhesion through early development. It is thought to protect and lubricate the embryo, stabilize the blastomeres during morphogenesis, and regulate nutrient intake. The major constituent of the hyaline layer is the protein hyalin. This matrix has been found in echinoderms.